regulation of toll-like receptor 2 signaling pathway [GO:0034135] (biological process) Relationships: is a type of regulation of pattern recognition receptor signaling pathway [GO:0062207]; regulates toll-like receptor 2 signaling pathway [GO:0034134] Subtypes: negative regulation of toll-like receptor 2 signaling pathway [GO:0034136], positive regulation of toll-like receptor 2 signaling pathway [GO:0034137] Also known as: regulation of TLR2 signaling pathway, regulation of toll-like receptor 2 signalling pathway Definition: Any process that modulates the frequency, rate, or extent of toll-like receptor 2 signaling pathway. References: PMID:16551253, PMID:17328678 Sources: GOC:add